{
  "term_label": "G protein-coupled receptor signaling pathway, coupled to cyclic nucleotide second messenger",
  "gene_symbol": "CHRM5",
  "term_id": "GO:0007187",
  "gene": "UniProtKB:P08912",
  "gene_name": "Muscarinic acetylcholine receptor M5"
}